{
  "gene": "UniProtKB:O43187",
  "gene_name": "Interleukin-1 receptor-associated kinase-like 2",
  "term_label": "Unknown molecular function",
  "term_id": "UNKNOWN:0001",
  "gene_symbol": "IRAK2"
}